{
  "gene_symbol": "FBLL1",
  "term_label": "histone H2AQ104 methyltransferase activity",
  "gene": "UniProtKB:A6NHQ2",
  "term_id": "GO:1990259",
  "gene_name": "rRNA_tRNA 2'-O-methyltransferase fibrillarin-like protein 1"
}